regulation of cell wall polysaccharide catabolic process [GO:2000966] (biological process) Subtypes: regulation of plant-type cell wall cellulose catabolic process [GO:2000939], negative regulation of cell wall polysaccharide catabolic process [GO:2000967], positive regulation of cell wall polysaccharide catabolic process [GO:2000968], GO:2000994 Also known as: regulation of cell wall polysaccharide breakdown Relationships: is a type of GO:0010981; is a type of regulation of polysaccharide metabolic process [GO:0032881]; is a type of GO:0043470; regulates cell wall polysaccharide catabolic process [GO:0044347] Definition: Any process that modulates the frequency, rate or extent of cell wall polysaccharide catabolic process. Sources: GOC:mengo_curators